{
  "term_label": "Unknown molecular function",
  "gene_symbol": "GEMIN7",
  "term_id": "UNKNOWN:0001",
  "gene": "UniProtKB:Q9H840",
  "gene_name": "Gem-associated protein 7"
}